{
  "gene": "UniProtKB:Q96N22",
  "gene_symbol": "ZNF681",
  "term_id": "GO:0005634",
  "gene_name": "Zinc finger protein 681",
  "term_label": "nucleus"
}